response to auxin [GO:0009733] (BP) Sources: GOC:jl Relationships: is a type of response to hormone [GO:0009725] Subtypes: detection of auxin stimulus [GO:0009721], cellular response to auxin stimulus [GO:0071365], response to indolebutyric acid [GO:0080026] Definition: Any process that results in a change in state or activity of a cell or an organism (in terms of movement, secretion, enzyme production, gene expression, etc.) as a result of an auxin stimulus. Also known as: response to auxin stimulus